{
  "gene_symbol": "SEC22C",
  "gene": "UniProtKB:Q9BRL7",
  "term_id": "UNKNOWN:0003",
  "term_label": "Unknown cellular component",
  "gene_name": "Vesicle-trafficking protein SEC22c"
}